{
  "term_id": "UNKNOWN:0003",
  "gene_name": "Protein Dok-7",
  "gene_symbol": "DOK7",
  "gene": "UniProtKB:Q18PE1",
  "term_label": "Unknown cellular component"
}